enamidase activity [GO:0043792] (molecular function) Definition: Catalysis of the reaction: 1,4,5,6-tetrahydro-6-oxonicotinate + 2 H2O = 2-formylglutarate + NH4. Sources: EC:3.5.2.18, RHEA:17209 Also known as: 6-oxo-1,4,5,6-tetrahydronicotinate amidohydrolase activity Relationships: is a type of GO:0016812